{
  "term_label": "protein serine/threonine kinase activity",
  "gene_name": "Serine_threonine-protein kinase NLK",
  "gene": "UniProtKB:Q9UBE8",
  "term_id": "GO:0004674",
  "gene_symbol": "NLK"
}